global gene silencing by mRNA cleavage [GO:0098795] (biological process) References: PMID:15009896 Also known as: gene silencing by mRNA cleavage, mRNA cleavage involved in gene silencing, RNA interference, targeting of mRNA for destruction, mRNA destabilization-mediated gene silencing, targeting of mRNA for destruction involved in RNA interference Relationships: is a type of post-transcriptional gene silencing [GO:0016441]; has part GO:0061157 Definition: A posttranscriptional gene silencing pathway that involves the cleavage of mRNAs in a non-gene-specific manner.